{
  "term_label": "nuclear-transcribed mRNA catabolic process, nonsense-mediated decay",
  "gene": "UniProtKB:Q9NPJ4",
  "term_id": "GO:0000184",
  "gene_name": "Proline-rich nuclear receptor coactivator 2",
  "gene_symbol": "PNRC2"
}